{
  "gene_name": "Alpha_beta hydrolase domain-containing protein 17C",
  "term_label": "endosome membrane",
  "gene": "UniProtKB:Q6PCB6",
  "gene_symbol": "ABHD17C",
  "term_id": "GO:0010008"
}